{
  "term_label": "nucleolus",
  "gene": "UniProtKB:Q9BVP2",
  "gene_name": "Guanine nucleotide-binding protein-like 3",
  "gene_symbol": "GNL3",
  "term_id": "GO:0005730"
}